{
  "term_label": "cytosol",
  "term_id": "GO:0005829",
  "gene": "UniProtKB:Q96N96",
  "gene_symbol": "SPATA13",
  "gene_name": "Spermatogenesis-associated protein 13"
}